microtubule sliding [GO:0051012] (biological process) Also known as: microtubule translocation Relationships: is a type of microtubule-based movement [GO:0007018] Definition: The movement of one microtubule along another microtubule. Subtypes: GO:0031534, plus-end directed microtubule sliding [GO:0031535] References: PMID:14557818, PMID:14614826